{
  "term_label": "kinetochore",
  "term_id": "GO:0000776",
  "gene": "UniProtKB:P49450",
  "gene_symbol": "CENPA",
  "gene_name": "Histone H3-like centromeric protein A"
}